{
  "gene_name": "Signal transducer and activator of transcription 2",
  "gene": "UniProtKB:P52630",
  "term_id": "GO:0043434",
  "term_label": "response to peptide hormone",
  "gene_symbol": "STAT2"
}